regulation of resting membrane potential [GO:0060075] (biological process) Relationships: is a type of regulation of membrane potential [GO:0042391] Sources: GOC:dph, GOC:ef, ISBN:0195088433 Also known as: regulation of resting potential Definition: Any process that modulates the establishment or extent of a resting potential, the electrical charge across the plasma membrane, with the interior of the cell negative with respect to the exterior. The resting potential is the membrane potential of a cell that is not stimulated to be depolarized or hyperpolarized.